{
  "term_label": "Arp2/3 protein complex",
  "term_id": "GO:0005885",
  "gene_name": "Actin-related protein 2_3 complex subunit 1B",
  "gene": "UniProtKB:O15143",
  "gene_symbol": "ARPC1B"
}